{
  "gene_symbol": "PIK3CG",
  "term_label": "phosphatidylinositol 3-kinase complex, class IA",
  "term_id": "GO:0005943",
  "gene": "UniProtKB:P48736",
  "gene_name": "Phosphatidylinositol 4,5-bisphosphate 3-kinase catalytic subunit gamma isoform"
}